{
  "gene_name": "Molecular chaperone MKKS",
  "gene_symbol": "MKKS",
  "gene": "UniProtKB:Q9NPJ1",
  "term_label": "cytoplasm",
  "term_id": "GO:0005737"
}